{
  "term_id": "UNKNOWN:0001",
  "gene_name": "Protein FAM180A",
  "term_label": "Unknown molecular function",
  "gene": "UniProtKB:Q6UWF9",
  "gene_symbol": "FAM180A"
}